microcystin transport [GO:1905431] (biological process) Definition: The directed movement of a microcystin into, out of or within a cell, or between cells, by means of some agent such as a transporter or pore. Relationships: is a type of amide transport [GO:0042886] References: PMID:26055554 Sources: GOC:TermGenie, GO_REF:0000065